{
  "term_label": "Unknown cellular component",
  "gene_name": "TBC1 domain family member 9",
  "term_id": "UNKNOWN:0003",
  "gene_symbol": "TBC1D9",
  "gene": "UniProtKB:Q6ZT07"
}